S-(hydroxymethyl)glutathione dehydrogenase (NAD+) activity [GO:0106322] (molecular function) Sources: RHEA:19985 Definition: Catalysis of the reaction: S-(hydroxymethyl)glutathione + NAD+ = S-formylglutathione + NADH + H+. Relationships: is a type of S-(hydroxymethyl)glutathione dehydrogenase [NAD(P)+] activity [GO:0051903]